sulfide oxidation, using sulfide dehydrogenase [GO:0070222] (biological process) Relationships: is a type of sulfide oxidation [GO:0019418] Sources: MetaCyc:PWY-5274 Also known as: sulphide oxidation, using sulfide dehydrogenase Definition: A sulfide oxidation process that proceeds via the reaction catalyzed by sulfide dehydrogenase.